{
  "term_id": "UNKNOWN:0003",
  "term_label": "Unknown cellular component",
  "gene": "UniProtKB:P61578",
  "gene_name": "Endogenous retrovirus group K member 16 Rec protein",
  "gene_symbol": "ERVK-16"
}